{
  "gene_name": "Zinc finger ZZ-type and EF-hand domain-containing protein 1",
  "gene_symbol": "ZZEF1",
  "term_label": "Unknown molecular function",
  "gene": "UniProtKB:O43149",
  "term_id": "UNKNOWN:0001"
}